undecaprenyl-diphosphatase activity [GO:0050380] (molecular function) References: PMID:18411271 Sources: RHEA:28094 Definition: Catalysis of the reaction: di-trans,octa-cis-undecaprenyl diphosphate + H2O = di-trans,octa-cis-undecaprenyl phosphate + H+ + phosphate. Relationships: is a type of polyprenyl diphosphate phosphatase activity [GO:0120556] Also known as: C(55)-isoprenyl diphosphatase activity, C(55)-isoprenyl pyrophosphatase activity, C55-isoprenyl diphosphatase activity, C55-isoprenyl pyrophosphatase activity, isoprenyl pyrophosphatase activity, undecaprenyl-diphosphate phosphohydrolase activity